9,15,9'-tri-cis-zeta-carotene isomerase activity [GO:0090471] (molecular function) Relationships: is a type of cis-trans isomerase activity [GO:0016859] Also known as: 9,15,9'-tricis-zeta-carotene cis-trans-isomerase Sources: RHEA:30967 Definition: Catalysis of the reaction: 9,9',15-tri-cis-zeta-carotene = 9,9'-di-cis-zeta-carotene.